{
  "gene_symbol": "TRIM59",
  "gene_name": "Tripartite motif-containing protein 59",
  "term_id": "GO:0043124",
  "gene": "UniProtKB:Q8IWR1",
  "term_label": "negative regulation of canonical NF-kappaB signal transduction"
}